{
  "gene": "UniProtKB:C9J798",
  "gene_symbol": "RASA4B",
  "term_id": "GO:0005096",
  "gene_name": "Ras GTPase-activating protein 4B",
  "term_label": "GTPase activator activity"
}